{
  "gene_symbol": "NPSR1",
  "term_id": "GO:0051281",
  "gene_name": "Neuropeptide S receptor",
  "gene": "UniProtKB:Q6W5P4",
  "term_label": "positive regulation of release of sequestered calcium ion into cytosol"
}